{
  "term_id": "GO:0004345",
  "gene_name": "Glucose-6-phosphate 1-dehydrogenase",
  "gene": "UniProtKB:P11413",
  "gene_symbol": "G6PD",
  "term_label": "glucose-6-phosphate dehydrogenase activity"
}